{
  "gene": "UniProtKB:Q14CX5",
  "term_label": "Unknown molecular function",
  "gene_symbol": "MFSD13A",
  "gene_name": "Transmembrane protein 180",
  "term_id": "UNKNOWN:0001"
}